{
  "gene_symbol": "SIPA1L3",
  "term_id": "GO:0003382",
  "gene": "UniProtKB:O60292",
  "gene_name": "Signal-induced proliferation-associated 1-like protein 3",
  "term_label": "epithelial cell morphogenesis"
}